regulation of melanin biosynthetic process [GO:0048021] (BP) Subtypes: negative regulation of melanin biosynthetic process [GO:0048022], positive regulation of melanin biosynthetic process [GO:0048023] Also known as: regulation of melanin anabolism, regulation of melanin biosynthesis, regulation of melanin formation, regulation of melanin synthesis Relationships: is a type of GO:1900376; regulates GO:0042438 Definition: Any process that alters the frequency, rate or extent of the chemical reactions and pathways resulting in the formation of melanin. Sources: GOC:jid